{
  "gene_symbol": "Q1T7F1",
  "gene_name": "Putative chemokine-related protein B42",
  "gene": "UniProtKB:Q1T7F1",
  "term_id": "UNKNOWN:0002",
  "term_label": "Unknown biological process"
}